protein import into chloroplast stroma [GO:0045037] (biological process) Definition: The targeting and import of proteins into the chloroplast stroma. Import depends on ATP hydrolysis catalyzed by stromal chaperones. Chloroplast stromal proteins, such as the S subunit of rubisco, have a N-terminal stromal-import sequence of about 44 amino acids which is cleaved from the protein precursor after import. Relationships: is a type of GO:0071806; is a type of establishment of protein localization to chloroplast [GO:0072596]; is a type of protein localization to chloroplast [GO:0072598] Sources: ISBN:0716731363 Also known as: chloroplast stroma protein import, protein transport into chloroplast stroma Regulation: regulated by regulation of protein import into chloroplast stroma [GO:1904215]; positively regulated by positive regulation of protein import into chloroplast stroma [GO:1904216]